regulation of peptidyl-serine phosphorylation of STAT protein [GO:0033139] (BP) Sources: GOC:mah Subtypes: negative regulation of peptidyl-serine phosphorylation of STAT protein [GO:0033140], positive regulation of peptidyl-serine phosphorylation of STAT protein [GO:0033141] Definition: Any process that modulates the frequency, rate or extent of the phosphorylation of a serine residue of a STAT (Signal Transducer and Activator of Transcription) protein. Also known as: regulation of serine phosphorylation of STAT3 protein Relationships: is a type of regulation of peptidyl-serine phosphorylation [GO:0033135]; regulates serine phosphorylation of STAT protein [GO:0042501]